{
  "gene_name": "TRPM8 channel associated factor 2C (Fragment)",
  "term_label": "plasma membrane",
  "term_id": "GO:0005886",
  "gene_symbol": "TCAF2C",
  "gene": "UniProtKB:A0A1B0GVM2"
}